response to nonylphenol [GO:1904147] (biological process) Definition: Any process that results in a change in state or activity of a cell or an organism (in terms of movement, secretion, enzyme production, gene expression, etc.) as a result of a nonylphenol stimulus. Relationships: is a type of GO:0042221 Subtypes: cellular response to nonylphenol [GO:1904148] References: PMID:19260726 Sources: GOC:TermGenie, GO_REF:0000071